{
  "term_label": "Unknown biological process",
  "gene": "UniProtKB:Q8IVF1",
  "gene_name": "NUT family member 2A",
  "term_id": "UNKNOWN:0002",
  "gene_symbol": "NUTM2A"
}